{
  "gene": "UniProtKB:Q8NI77",
  "term_id": "GO:1990023",
  "term_label": "mitotic spindle midzone",
  "gene_symbol": "KIF18A",
  "gene_name": "Kinesin-like protein KIF18A"
}